P2Y4 nucleotide receptor binding [GO:0031814] (molecular function) Also known as: P2Y4 nucleotide receptor ligand Relationships: is a type of G protein-coupled nucleotide receptor binding [GO:0031811] Sources: GOC:mah, GOC:nln Definition: Binding to a P2Y4 nucleotide receptor.